pyrimidine ribonucleotide metabolic process [GO:0009218] (BP) Sources: GOC:go_curators, ISBN:0198506732 Definition: The chemical reactions and pathways involving a pyrimidine ribonucleotide, a compound consisting of nucleoside (a pyrimidine base linked to a ribose sugar) esterified with a phosphate group at either the 3' or 5'-hydroxyl group of the sugar. Also known as: pyrimidine ribonucleotide metabolism Subtypes: GO:0009220, pyrimidine ribonucleotide catabolic process [GO:0009222], GO:0015954, CMP metabolic process [GO:0046035], GO:0046036, TDP metabolic process [GO:0046043], TMP metabolic process [GO:0046044], GO:0046046, GO:0046048, UMP metabolic process [GO:0046049], UTP metabolic process [GO:0046051], CDP metabolic process [GO:0046704] Relationships: is a type of pyrimidine nucleotide metabolic process [GO:0006220]; is a type of ribonucleotide metabolic process [GO:0009259]